{
  "gene": "UniProtKB:Q8IZL9",
  "gene_symbol": "CDK20",
  "term_id": "UNKNOWN:0002",
  "gene_name": "Cyclin-dependent kinase 20",
  "term_label": "Unknown biological process"
}